{
  "gene_symbol": "IFIT5",
  "term_label": "cytosol",
  "gene_name": "Interferon-induced protein with tetratricopeptide repeats 5",
  "gene": "UniProtKB:Q13325",
  "term_id": "GO:0005829"
}